{
  "gene_name": "Dystonin",
  "term_id": "GO:0005198",
  "gene": "UniProtKB:Q03001",
  "term_label": "structural molecule activity",
  "gene_symbol": "DST"
}